{
  "term_label": "reciprocal meiotic recombination",
  "gene_symbol": "RAD54B",
  "term_id": "GO:0007131",
  "gene": "UniProtKB:Q9Y620",
  "gene_name": "DNA repair and recombination protein RAD54B"
}